{
  "gene_name": "CKLF-like MARVEL transmembrane domain-containing protein 1",
  "gene_symbol": "CMTM1",
  "term_id": "GO:0016020",
  "gene": "UniProtKB:Q8IZ96",
  "term_label": "membrane"
}